{
  "term_id": "GO:0031012",
  "gene": "UniProtKB:Q8N158",
  "term_label": "extracellular matrix",
  "gene_symbol": "GPC2",
  "gene_name": "Glypican-2"
}